{
  "term_label": "ATP binding",
  "term_id": "GO:0005524",
  "gene_name": "Putative heat shock protein HSP 90-beta 2",
  "gene": "UniProtKB:Q58FF8",
  "gene_symbol": "HSP90AB2P"
}